{
  "gene_symbol": "CYBB",
  "gene": "UniProtKB:P04839",
  "gene_name": "Cytochrome b-245 heavy chain",
  "term_label": "NAD(P)H oxidase H2O2-forming activity",
  "term_id": "GO:0016174"
}